{
  "gene_symbol": "TIGD7",
  "term_label": "DNA binding",
  "gene": "UniProtKB:Q6NT04",
  "term_id": "GO:0003677",
  "gene_name": "Tigger transposable element-derived protein 7"
}